skeletal muscle hypertrophy [GO:0014734] (biological process) Relationships: is a type of striated muscle hypertrophy [GO:0014897]; is a type of skeletal muscle adaptation [GO:0043501] Regulation: regulated by GO:1904204; negatively regulated by GO:1904205; positively regulated by positive regulation of skeletal muscle hypertrophy [GO:1904206] Definition: The enlargement or overgrowth of all or part of an organ due to an increase in size (not length) of individual muscle fibers without cell division. In the case of skeletal muscle cells this happens due to the additional synthesis of sarcomeric proteins and assembly of myofibrils. Sources: GOC:mtg_muscle